{
  "gene": "UniProtKB:Q13901",
  "gene_name": "Nuclear nucleic acid-binding protein C1D",
  "gene_symbol": "C1D",
  "term_label": "DNA binding",
  "term_id": "GO:0003677"
}